{
  "gene": "UniProtKB:P11532",
  "gene_symbol": "DMD",
  "term_id": "GO:0007519",
  "gene_name": "Dystrophin",
  "term_label": "skeletal muscle tissue development"
}